{
  "term_label": "endoplasmic reticulum",
  "gene_symbol": "PIGW",
  "gene": "UniProtKB:Q7Z7B1",
  "term_id": "GO:0005783",
  "gene_name": "Phosphatidylinositol-glycan biosynthesis class W protein"
}